{
  "gene_symbol": "KCNQ5",
  "term_label": "voltage-gated potassium channel activity",
  "gene_name": "Potassium voltage-gated channel subfamily KQT member 5",
  "gene": "UniProtKB:Q9NR82",
  "term_id": "GO:0005249"
}